{
  "term_id": "UNKNOWN:0003",
  "term_label": "Unknown cellular component",
  "gene_name": "G-protein coupled receptor 78",
  "gene": "UniProtKB:Q96P69",
  "gene_symbol": "GPR78"
}